{
  "gene_symbol": "EYA4",
  "gene": "UniProtKB:O95677",
  "term_label": "protein tyrosine phosphatase activity",
  "term_id": "GO:0004725",
  "gene_name": "Eyes absent homolog 4"
}